{
  "gene": "UniProtKB:Q9UHL4",
  "term_label": "dipeptidyl-peptidase activity",
  "term_id": "GO:0008239",
  "gene_symbol": "DPP7",
  "gene_name": "Dipeptidyl peptidase 2"
}